{
  "gene": "UniProtKB:Q9NV39",
  "gene_symbol": "PRR34",
  "term_label": "Unknown biological process",
  "gene_name": "Proline-rich protein 34",
  "term_id": "UNKNOWN:0002"
}